negative regulation of arabinoxylan-containing compound catabolic process [GO:2000922] (biological process) Subtypes: negative regulation of glucuronoarabinoxylan catabolic process [GO:2000919] Sources: GOC:mengo_curators Relationships: is_a regulation of arabinoxylan-containing compound catabolic process [GO:2000921]; is a type of negative regulation of xylan catabolic process [GO:2001001]; negatively regulates arabinoxylan-containing compound catabolic process [GO:2000888] Definition: Any process that stops, prevents or reduces the frequency, rate or extent of arabinoxylan-containing compound catabolic process. Also known as: negative regulation of arabinoxylan catabolism